diaminobutyrate acetyltransferase activity [GO:0033816] (molecular function) Relationships: is a type of GO:0016407 Sources: EC:2.3.1.178, RHEA:16901 Also known as: 2,4-diaminobutanoate acetyltransferase activity, DAB acetyltransferase activity, DABA acetyltransferase activity, DABAcT, EctA, L-2,4-diaminobutanoate acetyltransferase activity, L-2,4-diaminobutyrate acetyltransferase activity, acetyl-CoA:L-2,4-diaminobutanoate 4-N-acetyltransferase activity, acetyl-CoA:L-2,4-diaminobutanoate N4-acetyltransferase activity, diaminobutyric acid acetyltransferase activity Definition: Catalysis of the reaction: L-2,4-diaminobutyrate + acetyl-CoA = N(4)-acetyl-L-2,4-diaminobutyrate + CoA + H+.